{
  "gene_name": "Short transient receptor potential channel 5",
  "term_label": "inositol 1,4,5 trisphosphate binding",
  "gene": "UniProtKB:Q9UL62",
  "term_id": "GO:0070679",
  "gene_symbol": "TRPC5"
}